cytosine C-5 DNA demethylase activity [GO:0051747] (molecular function) Relationships: is a type of hydrolase activity [GO:0016787]; is a type of DNA demethylase activity [GO:0035514] References: PMID:10050851 Also known as: DNA demethylase activity, hydrolytic DNA demethylase activity, DNA methyltransferase activity acting on cytosine C-5 Definition: Catalysis of the reaction: methyl-dCpdG DNA + H2O = dCpdG DNA + methanol. This reaction is the hydrolytic removal of the methyl group on the 5 position of cytosine in DNA.